{
  "term_id": "GO:0004984",
  "gene_name": "Olfactory receptor 8S1",
  "gene": "UniProtKB:Q8NH09",
  "term_label": "olfactory receptor activity",
  "gene_symbol": "OR8S1"
}